{
  "gene_symbol": "GARIN1B",
  "gene_name": "Golgi-associated RAB2 interactor protein 1B",
  "term_label": "Unknown molecular function",
  "gene": "UniProtKB:Q96KD3",
  "term_id": "UNKNOWN:0001"
}